{
  "gene_name": "Cadherin-2",
  "term_id": "GO:0043005",
  "gene": "UniProtKB:P19022",
  "gene_symbol": "CDH2",
  "term_label": "neuron projection"
}